{
  "gene_name": "Tubulin alpha-3D chain",
  "gene": "UniProtKB:P0DPH8",
  "gene_symbol": "TUBA3D",
  "term_id": "GO:0000278",
  "term_label": "mitotic cell cycle"
}